{
  "gene_name": "Heat shock protein 75 kDa, mitochondrial",
  "gene_symbol": "TRAP1",
  "term_id": "GO:0005743",
  "gene": "UniProtKB:Q12931",
  "term_label": "mitochondrial inner membrane"
}